{
  "gene_name": "Volume-regulated anion channel subunit LRRC8E",
  "gene": "UniProtKB:Q6NSJ5",
  "gene_symbol": "LRRC8E",
  "term_id": "GO:0098656",
  "term_label": "monoatomic anion transmembrane transport"
}